neuromuscular junction of somatic muscle myotube [GO:0098524] (cellular component) Definition: A neuromuscular junction in which the target muscle cell is a somatic muscle myotube, such as an arthropod somatic muscle cell. Sources: GOC:dos Relationships: is a type of neuromuscular junction of myotube [GO:0098523]; is a type of GO:0098527 Subtypes: excitatory neuromuscular junction of somatic myotube [GO:0098525], GO:0098526